activin receptor activity, type I [GO:0016361] (molecular function) Also known as: type I activin receptor activity References: PMID:8622651 Sources: GOC:mah Definition: Combining with activin-bound type II activin receptor to initiate a change in cell activity; upon binding, acts as a downstream transducer of activin signals. Relationships: is_a GO:0017002